{
  "gene": "UniProtKB:Q6NZY4",
  "gene_symbol": "ZCCHC8",
  "term_label": "RNA processing",
  "gene_name": "Zinc finger CCHC domain-containing protein 8",
  "term_id": "GO:0006396"
}